mitochondrial tRNA pseudouridine(27/28) synthase activity [GO:0160153] (MF) Definition: Catalysis of the reaction: uridine(27/28) in mitochondrial tRNA = pseudouridine(27/28) in mitochondrial tRNA. Relationships: is_a tRNA pseudouridine synthase activity [GO:0106029] Sources: EC:5.4.99.44